{
  "gene": "UniProtKB:Q9ULM0",
  "gene_name": "Pleckstrin homology domain-containing family H member 1",
  "term_id": "UNKNOWN:0002",
  "gene_symbol": "PLEKHH1",
  "term_label": "Unknown biological process"
}